{
  "term_label": "peroxisomal matrix",
  "term_id": "GO:0005782",
  "gene": "UniProtKB:O95822",
  "gene_symbol": "MLYCD",
  "gene_name": "Malonyl-CoA decarboxylase, mitochondrial"
}